{
  "gene_symbol": "TRIM68",
  "term_label": "innate immune response",
  "gene_name": "E3 ubiquitin-protein ligase TRIM68",
  "term_id": "GO:0045087",
  "gene": "UniProtKB:Q6AZZ1"
}